{
  "gene_symbol": "EEIG1",
  "gene_name": "Early estrogen-induced gene 1 protein",
  "gene": "UniProtKB:Q5T9C2",
  "term_id": "UNKNOWN:0002",
  "term_label": "Unknown biological process"
}